metanephric interstitial fibroblast fate commitment [GO:0072260] (biological process) Definition: The process in which the developmental fate of a cell becomes restricted such that it will develop into a metanephric interstitial fibroblast. Sources: GOC:mtg_kidney_jan10 Also known as: metanephros interstitial cell fate commitment Relationships: is a type of GO:0072153; is part of GO:0072258